{
  "gene_name": "Glutamate receptor ionotropic, delta-2",
  "gene": "UniProtKB:O43424",
  "term_id": "GO:0004971",
  "term_label": "AMPA glutamate receptor activity",
  "gene_symbol": "GRID2"
}